{
  "term_label": "sulfation",
  "gene": "UniProtKB:Q06520",
  "term_id": "GO:0051923",
  "gene_symbol": "SULT2A1",
  "gene_name": "Sulfotransferase 2A1"
}